{
  "gene": "UniProtKB:Q96NY7",
  "gene_name": "Chloride intracellular channel protein 6",
  "term_label": "Unknown biological process",
  "gene_symbol": "CLIC6",
  "term_id": "UNKNOWN:0002"
}